{
  "term_label": "extracellular space",
  "gene_name": "Serpin B10",
  "gene": "UniProtKB:P48595",
  "term_id": "GO:0005615",
  "gene_symbol": "SERPINB10"
}